{
  "gene_name": "Transmembrane protein 52B",
  "gene": "UniProtKB:Q4KMG9",
  "term_id": "UNKNOWN:0002",
  "term_label": "Unknown biological process",
  "gene_symbol": "TMEM52B"
}